{
  "gene_name": "Beta-tectorin",
  "term_label": "extracellular space",
  "gene": "UniProtKB:Q96PL2",
  "gene_symbol": "TECTB",
  "term_id": "GO:0005615"
}